{
  "gene_symbol": "PCDHA3",
  "term_label": "cell adhesion molecule binding",
  "gene_name": "Protocadherin alpha-3",
  "gene": "UniProtKB:Q9Y5H8",
  "term_id": "GO:0050839"
}